rRNA (uridine-2'-O-)-methyltransferase activity [GO:0008650] (molecular function) Definition: Catalysis of the reaction: a uridine in rRNA + S-adenosyl-L-methionine = a 2'-O-methyluridine in rRNA + S-adenosyl-L-homocysteine + H+. Sources: RHEA:54152 Relationships: is a type of rRNA (uridine) methyltransferase activity [GO:0016436]; is a type of GO:0062105